{
  "gene": "UniProtKB:P55210",
  "term_id": "GO:0043525",
  "gene_name": "Caspase-7",
  "term_label": "positive regulation of neuron apoptotic process",
  "gene_symbol": "CASP7"
}